{
  "term_label": "extracellular space",
  "gene_symbol": "WFDC1",
  "gene_name": "WAP four-disulfide core domain protein 1",
  "gene": "UniProtKB:Q9HC57",
  "term_id": "GO:0005615"
}